{
  "gene_symbol": "WASF2",
  "gene": "UniProtKB:Q9Y6W5",
  "term_label": "protein kinase A regulatory subunit binding",
  "term_id": "GO:0034237",
  "gene_name": "Actin-binding protein WASF2"
}